posterior mRNA localization involved in anterior/posterior axis specification [GO:0060814] (biological process) Relationships: is a type of intracellular mRNA localization involved in anterior/posterior axis specification [GO:0060811] Also known as: posterior mRNA localisation involved in anterior/posterior axis specification Definition: Any process in which a mRNA is transported to and maintained in the oocyte and/or syncytial embryo contributing to the specification of the anterior/posterior axis. Sources: GOC:dph, GOC:sdb_2009, GOC:tb